{
  "term_id": "GO:0031663",
  "gene_name": "Interleukin-1 receptor-associated kinase 3",
  "gene_symbol": "IRAK3",
  "term_label": "lipopolysaccharide-mediated signaling pathway",
  "gene": "UniProtKB:Q9Y616"
}